{
  "gene_symbol": "TRAJ33",
  "gene_name": "T cell receptor alpha joining 33 (Fragment)",
  "gene": "UniProtKB:A0A075B6W3",
  "term_label": "Unknown biological process",
  "term_id": "UNKNOWN:0002"
}